{
  "gene": "UniProtKB:Q9NQ60",
  "term_id": "GO:0002081",
  "gene_symbol": "EQTN",
  "gene_name": "Equatorin",
  "term_label": "outer acrosomal membrane"
}